{
  "gene": "UniProtKB:Q96SJ8",
  "term_id": "GO:0005886",
  "gene_symbol": "TSPAN18",
  "term_label": "plasma membrane",
  "gene_name": "Tetraspanin-18"
}